{
  "gene_name": "Immunoglobulin lambda variable 1-44",
  "term_label": "immune response",
  "gene": "UniProtKB:P01699",
  "gene_symbol": "IGLV1-44",
  "term_id": "GO:0006955"
}